{
  "gene_name": "Protein ABHD12B",
  "term_id": "GO:0052651",
  "term_label": "monoacylglycerol catabolic process",
  "gene": "UniProtKB:Q7Z5M8",
  "gene_symbol": "ABHD12B"
}